{
  "term_id": "GO:0004930",
  "gene_name": "Adhesion G-protein coupled receptor G1",
  "gene_symbol": "ADGRG1",
  "gene": "UniProtKB:Q9Y653",
  "term_label": "G protein-coupled receptor activity"
}